{
  "term_id": "GO:0000122",
  "gene_symbol": "MAGEB5",
  "gene": "UniProtKB:Q9BZ81",
  "term_label": "negative regulation of transcription by RNA polymerase II",
  "gene_name": "Melanoma-associated antigen B5"
}